{
  "gene": "UniProtKB:Q8N5I3",
  "term_label": "Unknown molecular function",
  "gene_name": "Potassium channel regulatory protein",
  "term_id": "UNKNOWN:0001",
  "gene_symbol": "KCNRG"
}